{
  "term_label": "Unknown molecular function",
  "gene": "UniProtKB:A0A1B0GUZ9",
  "term_id": "UNKNOWN:0001",
  "gene_name": "Uncharacterized protein",
  "gene_symbol": "A0A1B0GUZ9"
}